positive regulation of 3'-UTR-mediated mRNA stabilization [GO:1905870] (biological process) Relationships: is a type of GO:0010628; is a type of regulation of 3'-UTR-mediated mRNA stabilization [GO:1905868]; RO_0002213 GO:0070935 Also known as: positive regulation of 3'-untranslated region-mediated mRNA stabilization, up regulation of 3'-UTR-mediated mRNA stabilization, up regulation of 3'-untranslated region-mediated mRNA stabilization, up-regulation of 3'-UTR-mediated mRNA stabilization, up-regulation of 3'-untranslated region-mediated mRNA stabilization, upregulation of 3'-UTR-mediated mRNA stabilization, upregulation of 3'-untranslated region-mediated mRNA stabilization, activation of 3'-UTR-mediated mRNA stabilization, activation of 3'-untranslated region-mediated mRNA stabilization Definition: Any process that activates or increases the frequency, rate or extent of 3'-UTR-mediated mRNA stabilization. References: PMID:19737525 Sources: GOC:TermGenie, GO_REF:0000058